{
  "gene_symbol": "GRM6",
  "term_label": "plasma membrane",
  "term_id": "GO:0005886",
  "gene": "UniProtKB:O15303",
  "gene_name": "Metabotropic glutamate receptor 6"
}